{
  "gene_name": "Peptidyl-prolyl cis-trans isomerase A-like 4E",
  "gene_symbol": "PPIAL4E",
  "term_label": "protein folding",
  "gene": "UniProtKB:A0A075B759",
  "term_id": "GO:0006457"
}